{
  "gene_symbol": "UBE4B",
  "gene": "UniProtKB:O95155",
  "gene_name": "Ubiquitin conjugation factor E4 B",
  "term_label": "nucleus",
  "term_id": "GO:0005634"
}